{
  "gene": "UniProtKB:Q8NFP0",
  "term_id": "UNKNOWN:0002",
  "gene_symbol": "PXT1",
  "term_label": "Unknown biological process",
  "gene_name": "Peroxisomal testis-specific protein 1"
}